L-rhamnose mutarotase activity [GO:0062192] (molecular function) Definition: Catalysis of the reaction: alpha-L-rhamnose = beta-L-rhamnose. Sources: RHEA:25584 Relationships: is a type of GO:0016857